{
  "gene_symbol": "GPR162",
  "term_id": "UNKNOWN:0002",
  "gene_name": "Probable G-protein coupled receptor 162",
  "term_label": "Unknown biological process",
  "gene": "UniProtKB:Q16538"
}